{
  "term_id": "GO:0016592",
  "gene": "UniProtKB:Q96HR3",
  "term_label": "mediator complex",
  "gene_symbol": "MED30",
  "gene_name": "Mediator of RNA polymerase II transcription subunit 30"
}